{
  "term_id": "GO:0045202",
  "gene": "UniProtKB:Q9GZV7",
  "gene_name": "Hyaluronan and proteoglycan link protein 2",
  "gene_symbol": "HAPLN2",
  "term_label": "synapse"
}